{
  "term_id": "UNKNOWN:0003",
  "gene": "UniProtKB:Q0D2I5",
  "gene_symbol": "IFFO1",
  "gene_name": "Non-homologous end joining factor IFFO1",
  "term_label": "Unknown cellular component"
}